lateral root branching [GO:0080181] (biological process) Relationships: is a type of morphogenesis of a branching structure [GO:0001763]; is part of GO:0010102 Definition: Any process involved in the formation of branches in lateral roots. Sources: GOC:tb